{
  "gene_symbol": "C6orf136",
  "gene_name": "Uncharacterized protein C6orf136",
  "gene": "UniProtKB:Q5SQH8",
  "term_id": "UNKNOWN:0003",
  "term_label": "Unknown cellular component"
}